{
  "term_id": "GO:0005826",
  "gene": "UniProtKB:Q9BST9",
  "term_label": "actomyosin contractile ring",
  "gene_symbol": "RTKN",
  "gene_name": "Rhotekin"
}